{
  "gene_symbol": "KCNK6",
  "term_id": "GO:0015271",
  "term_label": "outward rectifier potassium channel activity",
  "gene": "UniProtKB:Q9Y257",
  "gene_name": "Potassium channel subfamily K member 6"
}